{
  "term_label": "microtubule cytoskeleton organization",
  "gene_name": "Tubulin delta chain",
  "term_id": "GO:0000226",
  "gene": "UniProtKB:Q9UJT1",
  "gene_symbol": "TUBD1"
}